symbiont-mediated disruption of host focal adhesion [GO:0141029] (biological process) Relationships: is a type of GO:0052008 Definition: A process in which a symbiont alters or subverts focal adhesion in its host. The host is defined as the larger of the organisms involved in a symbiotic interaction. References: PMID:19489119, PMID:24573681, PMID:24905543 Also known as: disruption by symbiont of host focal adhesion